regulation of leukocyte mediated immunity [GO:0002703] (biological process) Also known as: regulation of immune cell mediated immunity, regulation of leucocyte mediated immunity Subtypes: regulation of leukocyte mediated cytotoxicity [GO:0001910], negative regulation of leukocyte mediated immunity [GO:0002704], positive regulation of leukocyte mediated immunity [GO:0002705], regulation of lymphocyte mediated immunity [GO:0002706], regulation of dendritic cell cytokine production [GO:0002730], regulation of myeloid leukocyte mediated immunity [GO:0002886] Definition: Any process that modulates the frequency, rate, or extent of leukocyte mediated immunity. Sources: GOC:add Relationships: is a type of regulation of immune effector process [GO:0002697]; RO_0002211 leukocyte mediated immunity [GO:0002443]